{
  "gene": "UniProtKB:Q8WYN0",
  "gene_symbol": "ATG4A",
  "gene_name": "Cysteine protease ATG4A",
  "term_id": "GO:0034727",
  "term_label": "piecemeal microautophagy of the nucleus"
}